4-carboxymuconolactone decarboxylase activity [GO:0047575] (molecular function) Definition: Catalysis of the reaction: (R)-2-(carboxymethyl)-5-oxo-2,5-dihydro-2-furoate + H+ = 5-oxo-4,5-dihydro-2-furylacetate + CO2. Relationships: is a type of GO:0016831 Sources: EC:4.1.1.44, RHEA:23348 Also known as: 4-carboxymonolactone carboxy-lyase activity, 4-carboxymuconolactone carboxy-lyase (4,5-dihydro-5-oxofuran-2-acetate-forming), 4-carboxymuconolactone carboxy-lyase activity, gamma-4-carboxymuconolactone decarboxylase activity